{
  "gene_symbol": "LEO1",
  "gene_name": "RNA polymerase-associated protein LEO1",
  "term_label": "positive regulation of transcription elongation by RNA polymerase II",
  "gene": "UniProtKB:Q8WVC0",
  "term_id": "GO:0032968"
}